{
  "term_id": "GO:0051015",
  "gene_symbol": "ACTN1",
  "term_label": "actin filament binding",
  "gene_name": "Alpha-actinin-1",
  "gene": "UniProtKB:P12814"
}